{
  "term_label": "cytoplasm",
  "gene_symbol": "PFDN6",
  "term_id": "GO:0005737",
  "gene_name": "Prefoldin subunit 6",
  "gene": "UniProtKB:O15212"
}